mannitol dehydrogenase activity [GO:0046029] (molecular function) Relationships: is_a oxidoreductase activity, acting on the CH-OH group of donors, NAD or NADP as acceptor [GO:0016616]; is a type of GO:0031320 Definition: Catalysis of the reaction: D-mannitol + NAD+ = D-mannose + H+ + NADH. Also known as: NAD-dependent mannitol dehydrogenase activity, MTD activity, mannitol:NAD+ 1-oxidoreductase activity Sources: RHEA:15029